{
  "term_label": "Unknown molecular function",
  "term_id": "UNKNOWN:0001",
  "gene_name": "Transportin-3",
  "gene_symbol": "TNPO3",
  "gene": "UniProtKB:Q9Y5L0"
}